{
  "gene_symbol": "PYCR1",
  "term_label": "L-proline biosynthetic process",
  "term_id": "GO:0055129",
  "gene": "UniProtKB:P32322",
  "gene_name": "Pyrroline-5-carboxylate reductase 1, mitochondrial"
}